{
  "gene_name": "Mitochondrial coenzyme A diphosphatase NUDT8",
  "term_id": "GO:0015938",
  "gene": "UniProtKB:Q8WV74",
  "gene_symbol": "NUDT8",
  "term_label": "coenzyme A catabolic process"
}